{
  "gene_symbol": "RUBCNL",
  "gene": "UniProtKB:Q9H714",
  "term_label": "phosphatidylinositol phosphate binding",
  "gene_name": "Protein associated with UVRAG as autophagy enhancer",
  "term_id": "GO:1901981"
}